{
  "gene": "UniProtKB:Q6P9G0",
  "term_id": "UNKNOWN:0003",
  "term_label": "Unknown cellular component",
  "gene_symbol": "CYB5D1",
  "gene_name": "Cytochrome b5 domain-containing protein 1"
}